{
  "term_id": "GO:0015386",
  "gene": "UniProtKB:Q6AI14",
  "gene_symbol": "SLC9A4",
  "gene_name": "Sodium_hydrogen exchanger 4",
  "term_label": "potassium:proton antiporter activity"
}